{
  "term_id": "UNKNOWN:0003",
  "gene": "UniProtKB:Q3LI67",
  "gene_symbol": "KRTAP6-3",
  "term_label": "Unknown cellular component",
  "gene_name": "Keratin-associated protein 6-3"
}